{
  "term_id": "GO:0005654",
  "term_label": "nucleoplasm",
  "gene_name": "SURP and G-patch domain-containing protein 1",
  "gene": "UniProtKB:Q8IWZ8",
  "gene_symbol": "SUGP1"
}